{
  "term_label": "DNA-binding transcription factor activity, RNA polymerase II-specific",
  "gene": "UniProtKB:O95409",
  "gene_symbol": "ZIC2",
  "term_id": "GO:0000981",
  "gene_name": "Zinc finger protein ZIC 2"
}